{
  "term_id": "GO:0050767",
  "gene": "UniProtKB:P50553",
  "term_label": "regulation of neurogenesis",
  "gene_symbol": "ASCL1",
  "gene_name": "Achaete-scute homolog 1"
}